{
  "gene_name": "Zinc finger protein 483",
  "term_id": "GO:0000981",
  "gene": "UniProtKB:Q8TF39",
  "term_label": "DNA-binding transcription factor activity, RNA polymerase II-specific",
  "gene_symbol": "ZNF483"
}